{
  "gene": "UniProtKB:Q8NGL0",
  "term_label": "odorant binding",
  "term_id": "GO:0005549",
  "gene_name": "Olfactory receptor 5L2",
  "gene_symbol": "OR5L2"
}